{
  "term_id": "GO:0010468",
  "gene": "UniProtKB:O15553",
  "gene_symbol": "MEFV",
  "gene_name": "Pyrin",
  "term_label": "regulation of gene expression"
}